lanosterol O-acyltransferase activity [GO:0034738] (molecular function) Sources: GOC:mah Definition: Catalysis of the reaction: acyl-CoA + lanosterol = CoA + lanosterol ester. Relationships: is a type of sterol O-acyltransferase activity [GO:0004772]